{
  "gene_name": "Dual specificity protein phosphatase 2",
  "term_id": "GO:0005737",
  "gene": "UniProtKB:Q05923",
  "term_label": "cytoplasm",
  "gene_symbol": "DUSP2"
}